neurexin family protein binding [GO:0042043] (MF) Also known as: neuroligin Definition: Binding to a neurexin, a synaptic cell surface protein related to latrotoxin receptor, laminin and agrin. Neurexins act as cell recognition molecules at nerve terminals. References: PMID:18923512 Sources: GOC:curators, GOC:pr Relationships: is_a signaling receptor binding [GO:0005102]